detection of brassinosteroid stimulus [GO:0009729] (biological process) Definition: The series of events in which a brassinosteroid stimulus is received by a cell and converted into a molecular signal. Sources: GOC:sm Also known as: perception of brassinosteroid stimulus Relationships: is a type of detection of hormone stimulus [GO:0009720]; is a type of response to brassinosteroid [GO:0009741]